{
  "term_id": "UNKNOWN:0001",
  "gene_symbol": "FAM120A2P",
  "gene_name": "Putative uncharacterized protein FAM120A2P",
  "term_label": "Unknown molecular function",
  "gene": "UniProtKB:Q5T035"
}